{
  "gene": "UniProtKB:P40394",
  "term_id": "GO:0008270",
  "gene_name": "All-trans-retinol dehydrogenase [NAD(+)] ADH7",
  "gene_symbol": "ADH7",
  "term_label": "zinc ion binding"
}